{
  "term_label": "innate immune response",
  "gene_symbol": "TRIM51",
  "term_id": "GO:0045087",
  "gene_name": "Tripartite motif-containing protein 51",
  "gene": "UniProtKB:Q9BSJ1"
}